{
  "term_label": "NAD binding",
  "gene_name": "Nucleoside diphosphate-linked moiety X motif 6",
  "gene": "UniProtKB:P53370",
  "term_id": "GO:0051287",
  "gene_symbol": "NUDT6"
}